{
  "gene_name": "Transmembrane gamma-carboxyglutamic acid protein 3",
  "gene_symbol": "PRRG3",
  "term_label": "blood coagulation",
  "gene": "UniProtKB:Q9BZD7",
  "term_id": "GO:0007596"
}